{
  "gene_name": "Sodium_calcium exchanger 2",
  "term_label": "postsynapse",
  "term_id": "GO:0098794",
  "gene_symbol": "SLC8A2",
  "gene": "UniProtKB:Q9UPR5"
}